{
  "gene_name": "Coiled-coil domain-containing protein 34",
  "term_id": "UNKNOWN:0002",
  "gene_symbol": "CCDC34",
  "gene": "UniProtKB:Q96HJ3",
  "term_label": "Unknown biological process"
}